regulation of aspartate secretion [GO:1904448] (biological process) Definition: Any process that modulates the frequency, rate or extent of aspartate secretion. Subtypes: GO:1904449, positive regulation of aspartate secretion [GO:1904450] References: PMID:2342602 Sources: GOC:TermGenie, GO_REF:0000058 Relationships: is a type of regulation of organic acid transport [GO:0032890]; is_a regulation of amino acid transport [GO:0051955]; is_a GO:1903530; regulates aspartate secretion [GO:0061528]